C-C motif chemokine 19 receptor activity [GO:0038117] (molecular function) References: PMID:15059845 Sources: GOC:signaling Relationships: is a type of C-C chemokine receptor activity [GO:0016493]; is part of chemokine (C-C motif) ligand 19 signaling pathway [GO:0038115]; has part GO:0035757 Also known as: CCL19 receptor activity Definition: Combining with the C-C motif chemokine 19 (CCL19) and transmitting the signal from one side of the membrane to the other to initiate a change in cell activity.